{
  "gene_name": "Mammaglobin-A",
  "term_id": "GO:0030521",
  "gene": "UniProtKB:Q13296",
  "gene_symbol": "SCGB2A2",
  "term_label": "androgen receptor signaling pathway"
}